fungal biofilm matrix [GO:0062040] (cellular component) References: PMID:27129222, PMID:28516088 Sources: GOC:BHF Relationships: is a type of biofilm matrix [GO:0062039] Definition: An extracellular matrix lying external to fungal cells. The fungal biofilm matrix consists of polysaccharides, proteins, lipids, and nucleic acids. Fungal biofilms mediate adherence to host tissues, and provide protection from host immune defenses.